{
  "term_id": "GO:0007020",
  "gene_symbol": "HAUS2",
  "gene_name": "HAUS augmin-like complex subunit 2",
  "gene": "UniProtKB:Q9NVX0",
  "term_label": "microtubule nucleation"
}